sulfur compound catabolic process [GO:0044273] (biological process) Sources: GOC:jl Subtypes: sulfur amino acid catabolic process [GO:0000098], glutathione catabolic process [GO:0006751], coenzyme A catabolic process [GO:0015938], S-glycoside catabolic process [GO:0016145], dibenzothiophene catabolic process [GO:0018896], parathion catabolic process [GO:0019339], S-adenosylhomocysteine catabolic process [GO:0019510], GO:0032323, fatty-acyl-CoA catabolic process [GO:0036115], penicillin catabolic process [GO:0042317], biotin catabolic process [GO:0042367], GO:0042725, pyochelin catabolic process [GO:0042865], 2-aminobenzenesulfonate catabolic process [GO:0046230], thiocyanate catabolic process [GO:0046265], toluene-4-sulfonate catabolic process [GO:0046269], GO:0046306, GO:0046356, S-adenosylmethionine catabolic process [GO:0050843], cephamycin C catabolic process [GO:1901117], cephalosporin C catabolic process [GO:1901267], succinyl-CoA catabolic process [GO:1901289], glutathione derivative catabolic process [GO:1901686], leukotriene D4 catabolic process [GO:1901749], benzoyl-CoA catabolic process [GO:1901788], 2-hydroxybenzoyl-CoA catabolic process [GO:1901886], dimethylsulfoniopropionate catabolic process [GO:1902087], 6-sulfoquinovose(1-) catabolic process [GO:1902777], GO:2001294, gliotoxin catabolic process [GO:2001309] Relationships: is a type of sulfur compound metabolic process [GO:0006790]; is a type of catabolic process [GO:0009056] Also known as: sulfur compound breakdown, sulfur compound catabolism, sulfur compound degradation, sulfur catabolic process, sulfur catabolism Definition: The chemical reactions and pathways resulting in the breakdown of compounds that contain sulfur, such as the amino acids methionine and cysteine or the tripeptide glutathione.